RNA polymerase transcription factor SL1 complex [GO:0005668] (cellular component) Also known as: TIF-IB, selectivity factor SL1 complex References: PMID:15691654 Definition: A RNA polymerase I-specific transcription factor complex that contains the TATA-box-binding protein (TBP) and at least three TBP-associated factors including proteins known in mammals as TAFI110, TAFI63 and TAFI48. Relationships: is a type of RNA polymerase I transcription regulator complex [GO:0000120]